{
  "gene_name": "T-box transcription factor TBX1",
  "gene": "UniProtKB:O43435",
  "term_label": "DNA-binding transcription factor activity, RNA polymerase II-specific",
  "gene_symbol": "TBX1",
  "term_id": "GO:0000981"
}